{
  "gene": "UniProtKB:C9JCN9",
  "term_id": "UNKNOWN:0001",
  "term_label": "Unknown molecular function",
  "gene_name": "Heat shock factor-binding protein 1-like protein 1",
  "gene_symbol": "HSBP1L1"
}